chemokine production [GO:0032602] (biological process) Subtypes: fractalkine production [GO:0032603], chemokine (C-X-C motif) ligand 9 production [GO:0035393], chemokine (C-C motif) ligand 6 production [GO:0035530], GO:0036392, chemokine (C-C motif) ligand 17 production [GO:0044809], monocyte chemotactic protein-1 production [GO:0071605], chemokine (C-C motif) ligand 4 production [GO:0071606], GO:0071607, GO:0071608, chemokine (C-C motif) ligand 5 production [GO:0071609], GO:0071610, GO:0071612, chemokine (C-C motif) ligand 22 production [GO:0071924], thymic stromal lymphopoietin production [GO:0071925], chemokine (C-C motif) ligand 11 production [GO:0071954], chemokine (C-X-C motif) ligand 1 production [GO:0072566], chemokine (C-X-C motif) ligand 2 production [GO:0072567], chemokine (C-C motif) ligand 19 production [GO:0097388], chemokine (C-C motif) ligand 21 production [GO:0097389], chemokine (C-X-C motif) ligand 12 production [GO:0097390], GO:0097391, chemokine (C-X-C motif) ligand 16 production [GO:0097392] Regulation: regulated by regulation of chemokine production [GO:0032642]; negatively regulated by GO:0032682; positively regulated by positive regulation of chemokine production [GO:0032722] References: PMID:12183377 Sources: GOC:BHF, GOC:rl, ISBN:0198506732, Wikipedia:Chemokine Relationships: is a type of cytokine production [GO:0001816] Also known as: chemokine anabolism, chemokine biosynthesis, chemokine formation, chemokine synthesis, chemokine biosynthetic process, chemokine metabolic process, chemokine secretion Definition: The appearance of a chemokine due to biosynthesis or secretion following a cellular stimulus, resulting in an increase in its intracellular or extracellular levels. All chemokines possess a number of conserved cysteine residues involved in intramolecular disulfide bond formation. Some chemokines are considered pro-inflammatory and can be induced during an immune response to recruit cells of the immune system to a site of infection, while others are considered homeostatic and are involved in controlling the migration of cells during normal processes of tissue maintenance or development. Chemokines are found in all vertebrates, some viruses and some bacteria.